{
  "term_label": "Unknown molecular function",
  "term_id": "UNKNOWN:0001",
  "gene_symbol": "APOC4",
  "gene_name": "Apolipoprotein C-IV",
  "gene": "UniProtKB:P55056"
}